{
  "gene_symbol": "IL15RA",
  "gene_name": "Interleukin-15 receptor subunit alpha",
  "term_label": "interleukin-15-mediated signaling pathway",
  "gene": "UniProtKB:Q13261",
  "term_id": "GO:0035723"
}